{
  "gene_symbol": "ANKRD61",
  "gene": "UniProtKB:A6NGH8",
  "term_id": "UNKNOWN:0003",
  "term_label": "Unknown cellular component",
  "gene_name": "Ankyrin repeat domain-containing protein 61"
}